{
  "term_id": "UNKNOWN:0003",
  "gene": "UniProtKB:Q5T3J3",
  "gene_name": "Ligand-dependent nuclear receptor-interacting factor 1",
  "gene_symbol": "LRIF1",
  "term_label": "Unknown cellular component"
}